olefinic compound biosynthetic process [GO:0120255] (BP) Relationships: is a type of biosynthetic process [GO:0009058]; is a type of olefinic compound metabolic process [GO:0120254] Sources: GOC:krc Definition: The chemical reactions and pathways resulting in the formation of an olefinic compound, any compound which contains a carbon-carbon double bond (aka C=C). Also known as: alkene substituted compound anabolic process, alkene substituted compound anabolism, alkene substituted compound biosynthesis, alkene substituted compound biosynthetic process, alkene substituted compound synthesis Subtypes: GO:0006701, GO:0009688, chalcone biosynthetic process [GO:0009715], cinnamic acid biosynthetic process [GO:0009800], cinnamic acid ester biosynthetic process [GO:0009802], stilbene biosynthetic process [GO:0009811], prenol biosynthetic process [GO:0016091], aldosterone biosynthetic process [GO:0032342], GO:0033495, sinapate biosynthetic process [GO:0033497], cortisol biosynthetic process [GO:0034651], GO:0042855, GO:0061370, vomitoxin biosynthetic process [GO:0106110], viridicatumtoxin biosynthetic process [GO:0140872], paxilline biosynthetic process [GO:0140873], andrastin A biosynthetic process [GO:0140876], chanoclavine-I aldehyde biosynthetic process [GO:1900569], olefin biosynthetic process [GO:1900674], terrequinone A biosynthetic process [GO:1900796], helvolic acid biosynthetic process [GO:1900812], (-)-secologanin biosynthetic process [GO:1900994], GO:1901366, neoxanthin biosynthetic process [GO:1901833], isopentenol biosynthetic process [GO:1902934], geraniol biosynthetic process [GO:1903448], GO:1903449, kojic acid biosynthetic process [GO:2001317]